palmitoyl-CoA 9-desaturase activity [GO:0032896] (molecular function) Also known as: palmitoyl-CoA delta9-desaturase activity Relationships: is a type of acyl-CoA desaturase activity [GO:0016215] Definition: Catalysis of the reaction: hexadecanoyl-CoA + 2 Fe(II)-[cytochrome b5] + O2 + 2 H(+) = (9Z)-hexadecenoyl-CoA + 2 Fe(III)-[cytochrome b5] + 2 H2O. References: PMID:16443825 Sources: RHEA:36931